{
  "gene_symbol": "SH3GL2",
  "term_label": "cytosol",
  "gene_name": "Endophilin-A1",
  "gene": "UniProtKB:Q99962",
  "term_id": "GO:0005829"
}